{
  "term_id": "GO:0000209",
  "term_label": "protein polyubiquitination",
  "gene_symbol": "CDC34",
  "gene": "UniProtKB:P49427",
  "gene_name": "Ubiquitin-conjugating enzyme E2 R1"
}